morphogenesis of an epithelial fold involved in embryonic heart tube formation [GO:0003152] (biological process) Definition: The morphogenetic process in which an epithelial sheet bends along a linear axis, contributing to embryonic heart tube formation. Sources: GOC:mtg_heart Relationships: is a type of embryonic morphogenesis [GO:0048598]; is a type of GO:0060571; is part of embryonic heart tube formation via epithelial folding [GO:0003145] Subtypes: heart rudiment involution [GO:0003320]